response to food [GO:0032094] (biological process) Subtypes: cellular response to food [GO:0071240] Definition: Any process that results in a change in state or activity of a cell or an organism (in terms of movement, secretion, enzyme production, gene expression, etc.) as a result of a food stimulus; food is anything which, when taken into the body, serves to nourish or build up the tissues or to supply body heat. Relationships: is a type of response to nutrient levels [GO:0031667]; is a type of response to chemical [GO:0042221] Sources: GOC:add, ISBN:0721601464 Regulation: RO_0002211 by regulation of response to food [GO:0032095]; RO_0002212 by negative regulation of response to food [GO:0032096]; positively regulated by positive regulation of response to food [GO:0032097]